{
  "gene_name": "Megakaryocyte and platelet inhibitory receptor G6b",
  "term_id": "GO:0007229",
  "gene": "UniProtKB:O95866",
  "gene_symbol": "MPIG6B",
  "term_label": "integrin-mediated signaling pathway"
}